{
  "term_id": "UNKNOWN:0001",
  "gene_symbol": "MRPL34",
  "gene_name": "Large ribosomal subunit protein bL34m",
  "gene": "UniProtKB:Q9BQ48",
  "term_label": "Unknown molecular function"
}